{
  "gene_symbol": "CAPN15",
  "term_label": "calcium-dependent cysteine-type endopeptidase activity",
  "gene": "UniProtKB:O75808",
  "gene_name": "Calpain-15",
  "term_id": "GO:0004198"
}